nucleus lagging edge [GO:0110093] (cellular component) Definition: The area of a motile nucleus furthest from the direction of movement. References: PMID:24335254 Sources: GOC:kmv Relationships: is a type of GO:0110165; is part of GO:0005634